positive regulation of defense response to virus by host [GO:0002230] (biological process) Relationships: is a type of GO:0050691 Sources: GOC:add, GOC:dph, GOC:tb, ISBN:0781735149 Definition: Any host process that results in the promotion of antiviral immune response mechanisms, thereby limiting viral replication. Also known as: positive regulation of antiviral response by host, up regulation of antiviral response by host, up-regulation of antiviral response by host, upregulation of antiviral response by host, activation of antiviral response by host, stimulation of antiviral response by host